{
  "term_label": "3',5'-cyclic-AMP phosphodiesterase activity",
  "gene_name": "Dual 3',5'-cyclic-AMP and -GMP phosphodiesterase 11A",
  "term_id": "GO:0004115",
  "gene": "UniProtKB:Q9HCR9",
  "gene_symbol": "PDE11A"
}